mitochondrial seryl-tRNA aminoacylation [GO:0070158] (biological process) Definition: The process of coupling serine to seryl-tRNA in a mitochondrion, catalyzed by seryl-tRNA synthetase. In tRNA aminoacylation, the amino acid is first activated by linkage to AMP and then transferred to either the 2'- or the 3'-hydroxyl group of the 3'-adenosine residue of the tRNA. Sources: GOC:mah, GOC:mcc Relationships: is a type of seryl-tRNA aminoacylation [GO:0006434]; is a type of tRNA aminoacylation for mitochondrial protein translation [GO:0070127]